{
  "gene": "UniProtKB:Q9H0V9",
  "term_id": "GO:0005537",
  "gene_name": "VIP36-like protein",
  "gene_symbol": "LMAN2L",
  "term_label": "D-mannose binding"
}